{
  "gene": "UniProtKB:O95248",
  "term_label": "membrane",
  "gene_name": "Myotubularin-related protein 5",
  "term_id": "GO:0016020",
  "gene_symbol": "SBF1"
}